bicarbonate:monoatomic anion antiporter activity [GO:0140829] (molecular function) Relationships: is a type of monoatomic anion transmembrane transporter activity [GO:0008509]; is_a bicarbonate transmembrane transporter activity [GO:0015106]; is a type of antiporter activity [GO:0015297] Subtypes: chloride:bicarbonate antiporter activity [GO:0140900] Also known as: bicarbonate:anion antiporter activity, hydrogencarbonate:monoatomic anion antiporter activity Definition: Enables the transfer of a solute or solutes from one side of a membrane to the other according to the reaction: solute(in) + HCO3-(out) = solute(out) + HCO3-(in). References: PMID:12440690